synaptic vesicle tethering involved in synaptic vesicle exocytosis [GO:0099069] (biological process) Definition: The initial, indirect interaction between a synaptic vesicle membrane and a the preseynaptic membrane active zone. This interaction is mediated by tethering factors (or complexes), which interact with both membranes. This process is distinct from and prior to synaptic vesicle priming and fusion. Sources: GOC:rn Relationships: is a type of vesicle tethering involved in exocytosis [GO:0090522]; is part of GO:0016081